{
  "gene_symbol": "PTGER1",
  "term_label": "positive regulation of cytosolic calcium ion concentration",
  "gene": "UniProtKB:P34995",
  "gene_name": "Prostaglandin E2 receptor EP1 subtype",
  "term_id": "GO:0007204"
}